{
  "gene_symbol": "PLOD1",
  "term_label": "extracellular space",
  "term_id": "GO:0005615",
  "gene_name": "Procollagen-lysine,2-oxoglutarate 5-dioxygenase 1",
  "gene": "UniProtKB:Q02809"
}